{
  "gene_name": "Serine protease HTRA2, mitochondrial",
  "gene": "UniProtKB:O43464",
  "gene_symbol": "HTRA2",
  "term_id": "GO:0005739",
  "term_label": "mitochondrion"
}